enterobactin transmembrane transporter activity [GO:0042931] (molecular function) Definition: Enables the directed movement of the siderochrome enterochelin, a cyclic trimer of 2, 3 dihydroxybenzoylserine from one side of a membrane to the other. Also known as: enterochelin transporter activity, enterobactin transporter activity Sources: GOC:jl Relationships: is a type of siderophore-iron transmembrane transporter activity [GO:0015343]; is part of enterobactin transport [GO:0042930]